{
  "term_id": "GO:0000049",
  "gene": "UniProtKB:Q68D06",
  "gene_name": "Schlafen family member 13",
  "term_label": "tRNA binding",
  "gene_symbol": "SLFN13"
}